{
  "gene": "UniProtKB:Q6ZN68",
  "term_id": "GO:0005637",
  "term_label": "nuclear inner membrane",
  "gene_symbol": "DPY19L2P2",
  "gene_name": "Putative C-mannosyltransferase DPY19L2P2"
}